{
  "gene_symbol": "RTF1",
  "gene": "UniProtKB:Q92541",
  "gene_name": "RNA polymerase-associated protein RTF1 homolog",
  "term_label": "Unknown molecular function",
  "term_id": "UNKNOWN:0001"
}